negative regulation of glycolytic fermentation to ethanol [GO:2001155] (biological process) Relationships: is a type of negative regulation of catabolic process [GO:0009895]; is a type of negative regulation of carbohydrate metabolic process [GO:0045912]; is a type of GO:0062014; is a type of GO:2001154; negatively regulates pyruvate fermentation to ethanol [GO:0019655] Definition: Any process that stops, prevents or reduces the frequency, rate or extent of glucose catabolic process to ethanol. Also known as: negative regulation of ethanol fermentation, negative regulation of glucose fermentation to ethanol Sources: GOC:obol